negative regulation of telomere single strand break repair [GO:1903824] (biological process) References: PMID:24374808 Sources: GOC:TermGenie, GO_REF:0000058 Relationships: is a type of negative regulation of single strand break repair [GO:1903517]; negatively regulates GO:1903823 Also known as: down regulation of single strand break repair in telomere, down regulation of telomere single strand break repair, down regulation of telomere single-strand break repair, down regulation of telomeric single strand break repair, down-regulation of single strand break repair in telomere, down-regulation of telomere single strand break repair, down-regulation of telomere single-strand break repair, down-regulation of telomeric single strand break repair, downregulation of single strand break repair in telomere, downregulation of telomere single strand break repair, downregulation of telomere single-strand break repair, downregulation of telomeric single strand break repair, negative regulation of single strand break repair in telomere, negative regulation of telomere single-strand break repair, negative regulation of telomeric single strand break repair, inhibition of single strand break repair in telomere, inhibition of telomere single strand break repair, inhibition of telomere single-strand break repair, inhibition of telomeric single strand break repair, down regulation of telomere SSBR, down-regulation of telomere SSBR, downregulation of telomere SSBR, inhibition of telomere SSBR, negative regulation of telomere SSBR Definition: Any process that stops, prevents or reduces the frequency, rate or extent of telomere single strand break repair.